abaxial cell fate specification [GO:0010158] (biological process) Sources: GOC:mg Relationships: is a type of cell fate specification [GO:0001708] Definition: The process in which a cell becomes capable of differentiating autonomously into an abaxial cell in an environment that is neutral with respect to the developmental pathway; upon specification, the cell fate can be reversed.